{
  "term_id": "GO:0140374",
  "gene_name": "Interferon-induced protein with tetratricopeptide repeats 3",
  "term_label": "antiviral innate immune response",
  "gene_symbol": "IFIT3",
  "gene": "UniProtKB:O14879"
}